{
  "term_id": "GO:0005634",
  "gene_name": "Core histone macro-H2A.1",
  "term_label": "nucleus",
  "gene": "UniProtKB:O75367",
  "gene_symbol": "MACROH2A1"
}